{
  "term_id": "GO:0016251",
  "gene_name": "TATA-box-binding protein-associated factor 11-like protein 10",
  "gene_symbol": "TAF11L10",
  "gene": "UniProtKB:P0DW14",
  "term_label": "RNA polymerase II general transcription initiation factor activity"
}